chondroitin B lyase activity [GO:0033999] (molecular function) Sources: EC:4.2.2.19 Also known as: dermatan sulfate lyase activity, ChnB, chonB, chondroitinase B activity Relationships: is a type of carbon-oxygen lyase activity, acting on polysaccharides [GO:0016837] Definition: Catalysis of the reaction: dermatan sulfate = n 4-deoxy-beta-D-gluc-4-enuronosyl-(1,3)-N-acetyl-D-galactosamine 4-sulfate. This reaction is the eliminative cleavage of dermatan sulfate containing 1,4-beta-D-hexosaminyl and 1,3-beta-D-glucurosonyl or 1,3-alpha-L-iduronosyl linkages to disaccharides containing 4-deoxy-beta-D-gluc-4-enuronosyl groups to yield a 4,5-unsaturated dermatan-sulfate disaccharide (DeltaUA-GalNAC-4S). Chondroitin sulfate B is also known as dermatan sulfate.